{
  "gene_symbol": "RND2",
  "gene_name": "Rho-related GTP-binding protein RhoN",
  "gene": "UniProtKB:P52198",
  "term_id": "GO:0007015",
  "term_label": "actin filament organization"
}